positive regulation of DNA-directed DNA polymerase activity [GO:1900264] (BP) Also known as: activation of duplicase, positive regulation of duplicase, up regulation of duplicase, up-regulation of duplicase, upregulation of duplicase, activation of DNA duplicase activity, activation of DNA nucleotidyltransferase (DNA-directed) activity, activation of DNA replicase activity, activation of DNA-dependent DNA polymerase activity, activation of deoxynucleoside-triphosphate:DNA deoxynucleotidyltransferase (DNA-directed) activity, activation of deoxyribonucleic acid duplicase activity, activation of deoxyribonucleic duplicase activity, positive regulation of DNA duplicase activity, positive regulation of DNA nucleotidyltransferase (DNA-directed) activity, positive regulation of DNA replicase activity, positive regulation of DNA-dependent DNA polymerase activity, positive regulation of deoxynucleoside-triphosphate:DNA deoxynucleotidyltransferase (DNA-directed) activity, positive regulation of deoxyribonucleic acid duplicase activity, positive regulation of deoxyribonucleic duplicase activity, up regulation of DNA duplicase activity, up regulation of DNA nucleotidyltransferase (DNA-directed) activity, up regulation of DNA replicase activity, up regulation of DNA-dependent DNA polymerase activity, up regulation of DNA-directed DNA polymerase activity, up regulation of deoxynucleoside-triphosphate:DNA deoxynucleotidyltransferase (DNA-directed) activity, up regulation of deoxyribonucleic acid duplicase activity, up regulation of deoxyribonucleic duplicase activity, up-regulation of DNA duplicase activity, up-regulation of DNA nucleotidyltransferase (DNA-directed) activity, up-regulation of DNA replicase activity, up-regulation of DNA-dependent DNA polymerase activity, up-regulation of DNA-directed DNA polymerase activity, up-regulation of deoxynucleoside-triphosphate:DNA deoxynucleotidyltransferase (DNA-directed) activity, up-regulation of deoxyribonucleic acid duplicase activity, up-regulation of deoxyribonucleic duplicase activity, upregulation of DNA duplicase activity, upregulation of DNA nucleotidyltransferase (DNA-directed) activity, upregulation of DNA replicase activity, upregulation of DNA-dependent DNA polymerase activity, upregulation of DNA-directed DNA polymerase activity, upregulation of deoxynucleoside-triphosphate:DNA deoxynucleotidyltransferase (DNA-directed) activity, upregulation of deoxyribonucleic acid duplicase activity, upregulation of deoxyribonucleic duplicase activity, activation of DNA polymerase I, activation of DNA polymerase II, activation of DNA polymerase III, activation of DNA polymerase V activity, activation of DNA polymerase alpha, activation of DNA polymerase beta, activation of DNA polymerase gamma, activation of DNA-directed DNA polymerase activity, activation of Klenow fragment, activation of Taq DNA polymerase, activation of Taq Pol I, activation of Tca DNA polymerase, activation of alpha DNA polymerase activity, activation of beta DNA polymerase activity, activation of delta DNA polymerase activity, activation of deoxyribonucleic polymerase I, activation of epsilon DNA polymerase activity, activation of eta DNA polymerase activity, activation of gamma DNA-directed DNA polymerase activity, activation of iota DNA polymerase activity, activation of kappa DNA polymerase activity, activation of lambda DNA polymerase activity, activation of mu DNA polymerase activity, activation of nu DNA polymerase activity, activation of sigma DNA polymerase activity, activation of theta DNA polymerase activity, activation of zeta DNA polymerase activity, positive regulation of DNA polymerase I, positive regulation of DNA polymerase II, positive regulation of DNA polymerase III, positive regulation of DNA polymerase V activity, positive regulation of DNA polymerase alpha, positive regulation of DNA polymerase beta, positive regulation of DNA polymerase gamma, positive regulation of Klenow fragment, positive regulation of Taq DNA polymerase, positive regulation of Taq Pol I, positive regulation of Tca DNA polymerase, positive regulation of alpha DNA polymerase activity, positive regulation of beta DNA polymerase activity, positive regulation of delta DNA polymerase activity, positive regulation of deoxyribonucleic polymerase I, positive regulation of epsilon DNA polymerase activity, positive regulation of eta DNA polymerase activity, positive regulation of gamma DNA-directed DNA polymerase activity, positive regulation of iota DNA polymerase activity, positive regulation of kappa DNA polymerase activity, positive regulation of lambda DNA polymerase activity, positive regulation of mu DNA polymerase activity, positive regulation of nu DNA polymerase activity, positive regulation of sigma DNA polymerase activity, positive regulation of theta DNA polymerase activity, positive regulation of zeta DNA polymerase activity, up regulation of DNA polymerase I, up regulation of DNA polymerase II, up regulation of DNA polymerase III, up regulation of DNA polymerase V activity, up regulation of DNA polymerase alpha, up regulation of DNA polymerase beta, up regulation of DNA polymerase gamma, up regulation of Klenow fragment, up regulation of Taq DNA polymerase, up regulation of Taq Pol I, up regulation of Tca DNA polymerase, up regulation of alpha DNA polymerase activity, up regulation of beta DNA polymerase activity, up regulation of delta DNA polymerase activity, up regulation of deoxyribonucleic polymerase I, up regulation of epsilon DNA polymerase activity, up regulation of eta DNA polymerase activity, up regulation of gamma DNA-directed DNA polymerase activity, up regulation of iota DNA polymerase activity, up regulation of kappa DNA polymerase activity, up regulation of lambda DNA polymerase activity, up regulation of mu DNA polymerase activity, up regulation of nu DNA polymerase activity, up regulation of sigma DNA polymerase activity, up regulation of theta DNA polymerase activity, up regulation of zeta DNA polymerase activity, up-regulation of DNA polymerase I, up-regulation of DNA polymerase II, up-regulation of DNA polymerase III, up-regulation of DNA polymerase V activity, up-regulation of DNA polymerase alpha, up-regulation of DNA polymerase beta, up-regulation of DNA polymerase gamma, up-regulation of Klenow fragment, up-regulation of Taq DNA polymerase, up-regulation of Taq Pol I, up-regulation of Tca DNA polymerase, up-regulation of alpha DNA polymerase activity, up-regulation of beta DNA polymerase activity, up-regulation of delta DNA polymerase activity, up-regulation of deoxyribonucleic polymerase I, up-regulation of epsilon DNA polymerase activity, up-regulation of eta DNA polymerase activity, up-regulation of gamma DNA-directed DNA polymerase activity, up-regulation of iota DNA polymerase activity, up-regulation of kappa DNA polymerase activity, up-regulation of lambda DNA polymerase activity, up-regulation of mu DNA polymerase activity, up-regulation of nu DNA polymerase activity, up-regulation of sigma DNA polymerase activity, up-regulation of theta DNA polymerase activity, up-regulation of zeta DNA polymerase activity, upregulation of DNA polymerase I, upregulation of DNA polymerase II, upregulation of DNA polymerase III, upregulation of DNA polymerase V activity, upregulation of DNA polymerase alpha, upregulation of DNA polymerase beta, upregulation of DNA polymerase gamma, upregulation of Klenow fragment, upregulation of Taq DNA polymerase, upregulation of Taq Pol I, upregulation of Tca DNA polymerase, upregulation of alpha DNA polymerase activity, upregulation of beta DNA polymerase activity, upregulation of delta DNA polymerase activity, upregulation of deoxyribonucleic polymerase I, upregulation of epsilon DNA polymerase activity, upregulation of eta DNA polymerase activity, upregulation of gamma DNA-directed DNA polymerase activity, upregulation of iota DNA polymerase activity, upregulation of kappa DNA polymerase activity, upregulation of lambda DNA polymerase activity, upregulation of mu DNA polymerase activity, upregulation of nu DNA polymerase activity, upregulation of sigma DNA polymerase activity, upregulation of theta DNA polymerase activity, upregulation of zeta DNA polymerase activity, activation of sequenase, positive regulation of sequenase, up regulation of sequenase, up-regulation of sequenase, upregulation of sequenase Sources: GOC:TermGenie Definition: Any process that activates or increases the frequency, rate or extent of DNA-directed DNA polymerase activity. Relationships: is a type of GO:0043085; is a type of regulation of transferase activity [GO:0051338]; is a type of positive regulation of DNA biosynthetic process [GO:2000573]; positively regulates DNA-directed DNA polymerase activity [GO:0003887]